{
  "gene": "UniProtKB:P07288",
  "term_id": "GO:0031638",
  "term_label": "zymogen activation",
  "gene_name": "Prostate-specific antigen",
  "gene_symbol": "KLK3"
}